{
  "gene_symbol": "TMEM108",
  "term_id": "GO:0005769",
  "gene": "UniProtKB:Q6UXF1",
  "gene_name": "Transmembrane protein 108",
  "term_label": "early endosome"
}